{
  "term_id": "GO:0002181",
  "term_label": "cytoplasmic translation",
  "gene": "UniProtKB:Q59GN2",
  "gene_symbol": "RPL39P5",
  "gene_name": "Putative ribosomal protein eL39-like 5"
}